{
  "gene_name": "Protein FAM83C",
  "gene": "UniProtKB:Q9BQN1",
  "term_id": "GO:0007165",
  "term_label": "signal transduction",
  "gene_symbol": "FAM83C"
}